voltage-gated potassium channel activity involved in AV node cell action potential repolarization [GO:0086086] (molecular function) Also known as: voltage-gated potassium channel activity involved in AV node cardiac muscle cell action potential repolarization, voltage-gated potassium channel activity involved in atrioventricular node cardiac muscle cell action potential Definition: Catalysis of the transmembrane transfer of a potassium ion by a voltage-gated channel through the plasma membrane of an AV node cardiac muscle cell contributing to the repolarization phase of an action potential. A voltage-gated channel is a channel whose open state is dependent on the voltage across the membrane in which it is embedded. Sources: GOC:BHF, GOC:mtg_cardiac_conduct_nov11 Relationships: is a type of GO:0086008; is part of membrane repolarization during AV node cell action potential [GO:0086049]